protein phosphopantetheinylation [GO:0018215] (biological process) Sources: GOC:ai Definition: The modification of a protein amino acid by phosphopantetheinylation. Subtypes: peptidyl-serine phosphopantetheinylation [GO:0018070] Relationships: is a type of GO:0036211 Also known as: protein amino acid phosphopantetheinylation